octadecene metabolic process [GO:1900681] (biological process) Relationships: is a type of olefin metabolic process [GO:1900673] Also known as: octadecene metabolism Sources: GOC:TermGenie, GOC:mengo_curators Definition: The chemical reactions and pathways involving octadecene. Subtypes: GO:1900682